trophectodermal cell proliferation [GO:0001834] (biological process) Definition: The proliferation of cells in the trophectoderm. Sources: GOC:dph, ISBN:0124020607, ISBN:0198542771 Also known as: trophectoderm cell proliferation Note: See also the Anatomical Dictionary for Mouse Development ontology terms 'TS4, trophectoderm ; EMAP:19', 'TS5, trophectoderm ; EMAP:28' and 'TS6, trophectoderm ; EMAP:39'. Relationships: is a type of GO:0008283; is part of blastocyst growth [GO:0001832] Regulation: regulated by regulation of trophectodermal cell proliferation [GO:1904073]; negatively regulated by negative regulation of trophectodermal cell proliferation [GO:1904074]; positively regulated by GO:1904075